afferent axon development in anterior lateral line nerve [GO:0048910] (biological process) Definition: The process whose specific outcome is the progression of an afferent axon in the anterior lateral line nerve over time from its formation to the mature structure. This process includes axonogenesis and pathfinding of the afferent axons in the anterior lateral line nerve. References: PMID:15018940 Relationships: is a type of GO:0048893; is part of anterior lateral line nerve development [GO:0048909]